regulation of nuclear mRNA surveillance of meiosis-specific transcripts [GO:0120270] (biological process) Subtypes: GO:0120271, positive regulation of nuclear mRNA surveillance of meiosis-specific transcripts [GO:0120272] Definition: Any process that modulates the rate, frequency, or extent of selective degradation of meiosis-specific nuclear transcribed transcripts during vegetative growth, by a mechanism that requires determinant of selective removal (DSR) sequences in the targeted mRNAs and involves a YTH family protein. References: PMID:24920274 Sources: GOC:krc Relationships: is a type of regulation of mRNA catabolic process [GO:0061013]; RO_0002211 GO:0033621 Also known as: regulation of nuclear-transcribed mRNA catabolic process, meiosis-specific transcripts